{
  "gene": "UniProtKB:P02760",
  "term_label": "cell surface",
  "term_id": "GO:0009986",
  "gene_name": "Protein AMBP",
  "gene_symbol": "AMBP"
}